white fat cell differentiation [GO:0050872] (biological process) References: PMID:12508945 Also known as: white adipocyte cell differentiation, white adipocyte differentiation Subtypes: white fat cell differentiation involved in mammary gland fat development [GO:0060642] Relationships: is a type of GO:0045444 Definition: The process in which a relatively unspecialized cell acquires specialized features of a white adipocyte, an animal connective tissue cell involved in energy storage. White adipocytes have cytoplasmic lipids arranged in a unique vacuole. Regulation: negatively regulated by negative regulation of white fat cell differentiation [GO:0160275]